{
  "gene_symbol": "POU2F2",
  "gene_name": "POU domain, class 2, transcription factor 2",
  "term_id": "GO:0000981",
  "gene": "UniProtKB:P09086",
  "term_label": "DNA-binding transcription factor activity, RNA polymerase II-specific"
}